{
  "term_id": "GO:0043235",
  "term_label": "receptor complex",
  "gene_name": "Vascular endothelial growth factor receptor 3",
  "gene_symbol": "FLT4",
  "gene": "UniProtKB:P35916"
}